ketone body biosynthetic process [GO:0046951] (biological process) Subtypes: acetoacetic acid biosynthetic process [GO:0043441] Relationships: is_a small molecule biosynthetic process [GO:0044283]; is a type of fatty acid derivative biosynthetic process [GO:1901570]; is a type of GO:1902224 Sources: ISBN:0198506732 Also known as: ketone body anabolism, ketone body biosynthesis, ketone body formation, ketone body synthesis Definition: The chemical reactions and pathways resulting in the formation of ketone bodies, any one of the three substances: acetoacetate, D-3-hydroxybutyrate (beta-hydroxybutyrate) or acetone. Biosynthesis involves the formation of hydroxymethylglutaryl-CoA, which is cleaved to acetate and acetyl-CoA.